ABC-type phosphonate transporter activity [GO:0015416] (MF) Relationships: is a type of ABC-type transporter activity [GO:0140359]; is part of organic phosphonate transport [GO:0015716] Definition: Enables the transfer of a solute or solutes from one side of a membrane to the other according to the reaction: ATP + H2O + phosphonate(out) = ADP + phosphate + phosphonate(in). A phosphonate is any salt, anion, or ester of phosphonic acid (HPO(OH)2). Sources: RHEA:18065 Also known as: organic phosphonate transmembrane transporter activity, phosphonate ABC transporter, ATPase-coupled alkylphosphonate transmembrane transporter activity, alkylphosphonate ABC transporter activity, alkylphosphonate transmembrane transporter activity, alkylphosphonate transmembrane-transporting ATPase activity, ATP phosphohydrolase (phosphonate-transporting), ATPase-coupled organic phosphonate transmembrane transporter activity, organic phosphonate transmembrane-transporting ATPase activity, phosphonate transporting ATPase activity, phosphonate-transporting ATPase activity